{
  "term_label": "DNA-binding transcription factor activity, RNA polymerase II-specific",
  "gene_symbol": "ZNF676",
  "gene_name": "Zinc finger protein 676",
  "gene": "UniProtKB:Q8N7Q3",
  "term_id": "GO:0000981"
}